{
  "term_id": "GO:0007186",
  "gene_symbol": "OR8G2P",
  "gene_name": "Putative olfactory receptor 8G2",
  "term_label": "G protein-coupled receptor signaling pathway",
  "gene": "UniProtKB:Q6IF36"
}